{
  "gene": "UniProtKB:P49590",
  "term_label": "mitochondrial translation",
  "term_id": "GO:0032543",
  "gene_name": "Histidine--tRNA ligase, mitochondrial",
  "gene_symbol": "HARS2"
}